{
  "gene_symbol": "OXTR",
  "term_label": "oxytocin receptor activity",
  "gene": "UniProtKB:P30559",
  "gene_name": "Oxytocin receptor",
  "term_id": "GO:0004990"
}